{
  "term_label": "DNA-binding transcription factor activity, RNA polymerase II-specific",
  "gene_name": "Krueppel-like factor 4",
  "gene": "UniProtKB:O43474",
  "gene_symbol": "KLF4",
  "term_id": "GO:0000981"
}